{
  "gene_symbol": "GALNT11",
  "gene": "UniProtKB:Q8NCW6",
  "term_label": "Notch binding",
  "gene_name": "Polypeptide N-acetylgalactosaminyltransferase 11",
  "term_id": "GO:0005112"
}